{
  "gene_symbol": "PDE5A",
  "term_id": "GO:0047555",
  "term_label": "3',5'-cyclic-GMP phosphodiesterase activity",
  "gene": "UniProtKB:O76074",
  "gene_name": "cGMP-specific 3',5'-cyclic phosphodiesterase"
}